single-species surface biofilm formation [GO:0090606] (biological process) Definition: A process in which microorganisms produce an extracellular matrix and form multicellular aggregates at an air-liquid interface. Relationships: is a type of single-species biofilm formation [GO:0044010]; is a type of surface biofilm formation [GO:0090604] Also known as: multicellular pellicle formation Sources: GOC:ml